{
  "term_id": "GO:0051177",
  "gene_name": "Shugoshin 2",
  "term_label": "meiotic sister chromatid cohesion",
  "gene": "UniProtKB:Q562F6",
  "gene_symbol": "SGO2"
}